induction of negative chemotaxis [GO:0050929] (biological process) Sources: GOC:ai Definition: Any process that initiates the directed movement of a motile cell or organism towards a lower concentration in a concentration gradient of a specific chemical. Relationships: is a type of positive regulation of negative chemotaxis [GO:0050924]